{
  "gene_symbol": "TSPAN18",
  "gene_name": "Tetraspanin-18",
  "term_id": "UNKNOWN:0002",
  "gene": "UniProtKB:Q96SJ8",
  "term_label": "Unknown biological process"
}